{
  "gene_symbol": "ZSCAN25",
  "term_id": "GO:0000978",
  "gene": "UniProtKB:Q6NSZ9",
  "term_label": "RNA polymerase II cis-regulatory region sequence-specific DNA binding",
  "gene_name": "Zinc finger and SCAN domain-containing protein 25"
}